{
  "gene_symbol": "IGKV1D-39",
  "gene_name": "Immunoglobulin kappa variable 1D-39",
  "gene": "UniProtKB:P04432",
  "term_label": "Unknown molecular function",
  "term_id": "UNKNOWN:0001"
}